ice binding [GO:0050825] (molecular function) Subtypes: antifreeze activity [GO:0016172], GO:0019833 Relationships: is_a GO:0036094 Sources: GOC:curators Definition: Binding to ice, water reduced to the solid state by cold temperature. It is a white or transparent colorless substance, crystalline, brittle, and viscoidal. Also known as: ice crystal binding, ice nucleation inhibitor activity